{
  "gene": "UniProtKB:Q96P20",
  "gene_name": "NACHT, LRR and PYD domains-containing protein 3",
  "gene_symbol": "NLRP3",
  "term_id": "GO:0140297",
  "term_label": "DNA-binding transcription factor binding"
}